{
  "term_label": "transcription initiation at RNA polymerase II promoter",
  "gene_name": "General transcription factor IIH subunit 3",
  "term_id": "GO:0006367",
  "gene": "UniProtKB:Q13889",
  "gene_symbol": "GTF2H3"
}